cellular response to L-dopa [GO:1904474] (biological process) References: PMID:25044243 Sources: GOC:TermGenie, GO_REF:0000071 Definition: Any process that results in a change in state or activity of a cell (in terms of movement, secretion, enzyme production, gene expression, etc.) as a result of a L-dopa stimulus. Relationships: is a type of cellular response to amino acid stimulus [GO:0071230]; is_a cellular response to oxygen-containing compound [GO:1901701]; is a type of cellular response to L-phenylalanine derivative [GO:1904387]; is a type of response to L-dopa [GO:1904473]